{
  "gene_name": "Ras-related protein Rab-21",
  "term_id": "GO:0003924",
  "gene": "UniProtKB:Q9UL25",
  "term_label": "GTPase activity",
  "gene_symbol": "RAB21"
}